{
  "term_label": "molecular adaptor activity",
  "gene": "UniProtKB:Q8TBH0",
  "gene_symbol": "ARRDC2",
  "term_id": "GO:0060090",
  "gene_name": "Arrestin domain-containing protein 2"
}